{
  "term_id": "GO:0005200",
  "term_label": "structural constituent of cytoskeleton",
  "gene_name": "Tubulin alpha-3E chain",
  "gene": "UniProtKB:Q6PEY2",
  "gene_symbol": "TUBA3E"
}